{
  "gene_name": "Beta-galactosidase",
  "gene": "UniProtKB:P16278",
  "term_label": "galactose catabolic process",
  "term_id": "GO:0019388",
  "gene_symbol": "GLB1"
}